sarcosine metabolic process [GO:1901052] (biological process) References: PMID:17951379 Sources: GOC:TermGenie, GOC:yaf Definition: The chemical reactions and pathways involving sarcosine. Relationships: is a type of modified amino acid metabolic process [GO:0006575]; is a type of GO:0170041; is a type of GO:1901605 Subtypes: sarcosine catabolic process [GO:1901053], GO:1901054 Also known as: sarcosine metabolism